{
  "gene_name": "Peptide-N(4)-(N-acetyl-beta-glucosaminyl)asparagine amidase",
  "gene": "UniProtKB:Q96IV0",
  "gene_symbol": "NGLY1",
  "term_id": "GO:0006516",
  "term_label": "glycoprotein catabolic process"
}